{
  "gene_symbol": "PI3",
  "gene": "UniProtKB:P19957",
  "term_id": "GO:0045087",
  "term_label": "innate immune response",
  "gene_name": "Elafin"
}